{
  "term_id": "GO:0000977",
  "gene_name": "Hypoxia-inducible factor 3-alpha",
  "gene": "UniProtKB:Q9Y2N7",
  "gene_symbol": "HIF3A",
  "term_label": "RNA polymerase II transcription regulatory region sequence-specific DNA binding"
}